{
  "gene_name": "Bone morphogenetic protein receptor type-1B",
  "gene": "UniProtKB:O00238",
  "gene_symbol": "BMPR1B",
  "term_label": "dorsal/ventral pattern formation",
  "term_id": "GO:0009953"
}